{
  "term_label": "positive regulation of transcription by RNA polymerase II",
  "gene_symbol": "GATA5",
  "term_id": "GO:0045944",
  "gene": "UniProtKB:Q9BWX5",
  "gene_name": "Transcription factor GATA-5"
}